ACC codon-amino acid adaptor activity [GO:0033438] (molecular function) Definition: A triplet codon-amino acid adaptor activity that recognizes an ACC codon. Sources: GOC:mah Relationships: is a type of triplet codon-amino acid adaptor activity [GO:0030533] Also known as: threonine tRNA Note: Note that in the standard genetic code, ACC codes for threonine.